{
  "term_label": "cytokine binding",
  "gene": "UniProtKB:P42702",
  "term_id": "GO:0019955",
  "gene_name": "Leukemia inhibitory factor receptor",
  "gene_symbol": "LIFR"
}